dorsal fin development [GO:0033337] (biological process) Sources: GOC:dgh Definition: The process whose specific outcome is the progression of the dorsal fin over time, from its formation to the mature structure. Relationships: is_a medial fin development [GO:0033338]